{
  "gene_symbol": "ACTR10",
  "gene_name": "Actin-related protein 10",
  "term_id": "GO:0098958",
  "term_label": "retrograde axonal transport of mitochondrion",
  "gene": "UniProtKB:Q9NZ32"
}